4-hydroxy-3-polyprenylbenzoate decarboxylase activity [GO:0008694] (molecular function) Also known as: 3-polyprenyl 4-hydroxybenzoate decarboxylase activity, 3-polyprenyl-4-hydroxybenzoate carboxy-lyase activity, PPHB decarboxylase activity, polyprenyl p-hydroxybenzoate decarboxylase activity, 3-octaprenyl-4-hydroxybenzoate carboxy-lyase activity, 3-octaprenyl-4-hydroxybenzoate decarboxylase activity, UbiD, UbiX Relationships: is a type of carboxy-lyase activity [GO:0016831] Definition: Catalysis of the reaction: a 4-hydroxy-3-(all-trans-polyprenyl)benzoate + H+ = a 2-(all-trans-polyprenyl)phenol + CO2. Sources: RHEA:41680